{
  "gene": "UniProtKB:O95867",
  "term_id": "UNKNOWN:0001",
  "gene_name": "Lymphocyte antigen 6 complex locus protein G6c",
  "term_label": "Unknown molecular function",
  "gene_symbol": "LY6G6C"
}